{
  "term_label": "microvillus",
  "gene_name": "Unconventional myosin-Ia",
  "term_id": "GO:0005902",
  "gene": "UniProtKB:Q9UBC5",
  "gene_symbol": "MYO1A"
}